atrazine catabolic process to isopropylamine [GO:0019624] (BP) Definition: The chemical reactions and pathways resulting in the breakdown of atrazine, a triazine ring-containing herbicide, into isopropylamine. Relationships: is_a GO:0019381 Sources: GOC:jl Also known as: atrazine breakdown to isopropylamine, atrazine degradation to isopropylamine